FMN reductase [NAD(P)H] activity [GO:0008752] (MF) Relationships: is a type of oxidoreductase activity, acting on the CH-NH group of donors, NAD or NADP as acceptor [GO:0016646] Also known as: FMN reductase activity, NAD(P)H dehydrogenase (FMN) activity, NAD(P)H-dependent FMN reductase activity, flavin mononucleotide reductase activity Definition: Catalysis of the reaction: FMNH2 + NAD(P)+ = FMN + NAD(P)H + H+. This reaction can utilize NADH and NADPH with similar reaction rates. Sources: EC:1.5.1.39 Subtypes: FMN reductase (NADPH) activity [GO:0052873], GO:0052874